{
  "gene_symbol": "CASP3",
  "gene_name": "Caspase-3",
  "gene": "UniProtKB:P42574",
  "term_id": "GO:0006508",
  "term_label": "proteolysis"
}